{
  "gene_name": "Interferon alpha-8",
  "gene_symbol": "IFNA8",
  "term_label": "adaptive immune response",
  "term_id": "GO:0002250",
  "gene": "UniProtKB:P32881"
}